RAM/MOR signaling [GO:0062200] (biological process) Definition: An intracellular signaling cascade that starts with the activation of S. cerevisiae Kic1p, which activate Mob2p and Cbk1p. Cbk1p phosphorylates Ace2p, which results in its nuclear translocation, where it regulates transcription of genes involved in polarity and morphogenesis. Relationships: is a type of intracellular signal transduction [GO:0035556] Also known as: RAM/MOR signaling pathway, morphogenesis Orb6 network, MOR signaling pathway, RAM signaling pathway References: PMID:15731009, PMID:16096637, PMID:20805322, PMID:20826805, PMID:21246752, PMID:22629372, PMID:23212898